{
  "term_id": "GO:0098978",
  "gene": "UniProtKB:Q9Y4K3",
  "gene_name": "TNF receptor-associated factor 6",
  "gene_symbol": "TRAF6",
  "term_label": "glutamatergic synapse"
}